{
  "gene_name": "WAS protein family homolog 6",
  "term_label": "Unknown molecular function",
  "term_id": "UNKNOWN:0001",
  "gene_symbol": "WASH6P",
  "gene": "UniProtKB:Q9NQA3"
}